dolichyl-phosphate-mannose-protein mannosyltransferase Pmt4p homodimer complex [GO:0097586] (CC) Also known as: dolichyl-phosphate-mannose-protein mannosyltransferase Pmt4p dimer, dolichyl-phosphate-mannose-protein mannosyltransferase Pmt4p-Pmt4p dimer complex, Pmt4p-Pmt4p complex References: PMID:12551906 Sources: GOC:bhm, GOC:jd Definition: A protein dimer complex that possesses dolichyl-phosphate-mannose-protein mannosyltransferase activity and, in S. cerevisiae, is composed of Pmt4p. Relationships: is a type of GO:0031502